{
  "gene_symbol": "RCAN1",
  "gene": "UniProtKB:P53805",
  "term_id": "GO:0019722",
  "term_label": "calcium-mediated signaling",
  "gene_name": "Calcipressin-1"
}